{
  "term_label": "transcription regulator inhibitor activity",
  "gene_name": "Mothers against decapentaplegic homolog 6",
  "gene": "UniProtKB:O43541",
  "gene_symbol": "SMAD6",
  "term_id": "GO:0140416"
}